{
  "term_label": "glutamate-tRNA ligase activity",
  "gene_symbol": "EARS2",
  "term_id": "GO:0004818",
  "gene": "UniProtKB:Q5JPH6",
  "gene_name": "Probable glutamate--tRNA ligase, mitochondrial"
}